{
  "term_label": "cytosol",
  "gene": "UniProtKB:O00182",
  "gene_name": "Galectin-9",
  "term_id": "GO:0005829",
  "gene_symbol": "LGALS9"
}